{
  "term_id": "GO:0009897",
  "gene": "UniProtKB:P15328",
  "gene_name": "Folate receptor alpha",
  "term_label": "external side of plasma membrane",
  "gene_symbol": "FOLR1"
}